response to hypobaric hypoxia [GO:1990910] (biological process) Relationships: is a type of GO:0001666 Definition: Any process that results in a change in state or activity of a cell or an organism (in terms of movement, secretion, enzyme production, gene expression, etc.) as a result of a stimulus indicating lowered oxygen tension combined with low atmospheric pressure. Hypoxia is defined as a decline in O2 levels below normoxic levels of 20.8 - 20.95% and hypobaric is defined as atmospheric pressure below 0.74 atm (greater than 2,500 m above sea level). References: PMID:24590457